calcium-induced calcium release activity involved in regulation of postsynaptic cytosolic calcium ion concentration [GO:1905058] (molecular function) Relationships: is a type of calcium-induced calcium release activity [GO:0048763]; is part of regulation of postsynaptic cytosolic calcium ion concentration [GO:0099566] Definition: Any calcium-induced calcium release activity that is involved in regulation of postsynaptic cytosolic calcium ion concentration. Subtypes: ryanodine-sensitive calcium-release channel activity involved in regulation of postsynaptic cytosolic calcium levels [GO:0098697] Also known as: calcium-induced calcium release activity involved in regulation of postsynaptic cytosolic calcium levels References: PMID:23639769 Sources: GOC:TermGenie, GO_REF:0000061